{
  "gene_name": "T-cell activation Rho GTPase-activating protein",
  "gene": "UniProtKB:Q8N103",
  "gene_symbol": "TAGAP",
  "term_label": "GTPase activator activity",
  "term_id": "GO:0005096"
}